{
  "term_id": "GO:0005776",
  "gene_name": "Ras-related protein Rab-23",
  "term_label": "autophagosome",
  "gene": "UniProtKB:Q9ULC3",
  "gene_symbol": "RAB23"
}